{
  "gene_name": "Vacuolar protein sorting-associated protein 4B",
  "gene_symbol": "VPS4B",
  "term_id": "GO:0007033",
  "gene": "UniProtKB:O75351",
  "term_label": "vacuole organization"
}